{
  "gene_symbol": "GAS6",
  "term_id": "GO:0048018",
  "gene": "UniProtKB:Q14393",
  "term_label": "receptor ligand activity",
  "gene_name": "Growth arrest-specific protein 6"
}